neural crest-derived cardiac glial cell differentiation [GO:0060951] (biological process) Definition: The process in which a neural crest cell acquires the specialized features of a glial cell of the heart. Sources: GOC:mtg_heart Relationships: is a type of cardiac glial cell differentiation [GO:0060950]